negative regulation of blood vessel endothelial cell differentiation [GO:0110059] (biological process) Definition: Any process that stops, prevents, or reduces the frequency, rate or extent of blood vessel endothelial cell differentiation. Subtypes: negative regulation of venous endothelial cell fate commitment [GO:2000788] Relationships: is a type of negative regulation of endothelial cell differentiation [GO:0045602]; is a type of regulation of blood vessel endothelial cell differentiation [GO:0110057]; negatively regulates blood vessel endothelial cell differentiation [GO:0060837] References: PMID:23072816 Sources: GOC:BHF, GOC:BHF_miRNA, GOC:rph